{
  "gene": "UniProtKB:A0A075B6H9",
  "term_id": "GO:0019814",
  "gene_name": "Immunoglobulin lambda variable 4-69",
  "gene_symbol": "IGLV4-69",
  "term_label": "immunoglobulin complex"
}